{
  "gene_symbol": "C4BPB",
  "term_label": "Unknown molecular function",
  "gene": "UniProtKB:P20851",
  "term_id": "UNKNOWN:0001",
  "gene_name": "C4b-binding protein beta chain"
}